phosphoglucomutase (glucose-cofactor) activity [GO:0047468] (molecular function) Relationships: is a type of GO:0004614 Definition: Catalysis of the reaction: glucose-1-phosphate = glucose-6-phosphate; using D-glucose as a cofactor. Also known as: alpha-D-glucose 1,6-phosphomutase (glucose-cofactor), glucose-1-phosphate phosphotransferase activity Sources: EC:5.4.2.5